{
  "term_label": "Unknown molecular function",
  "gene_symbol": "TRAV17",
  "term_id": "UNKNOWN:0001",
  "gene_name": "T cell receptor alpha variable 17",
  "gene": "UniProtKB:A0A0B4J275"
}